{
  "term_label": "endonucleolytic cleavage to generate mature 3'-end of SSU-rRNA from (SSU-rRNA, 5.8S rRNA, LSU-rRNA)",
  "gene": "UniProtKB:P63220",
  "gene_symbol": "RPS21",
  "gene_name": "Small ribosomal subunit protein eS21",
  "term_id": "GO:0000461"
}